N6-hydroxylysine O-acetyltransferase activity [GO:0050133] (molecular function) Relationships: is a type of GO:0016413 Also known as: N(6)-hydroxylysine acetylase activity, N6-hydroxylysine acetylase activity, N6-hydroxylysine:acetyl CoA N6-transacetylase activity, acetyl-CoA:6-N-hydroxy-L-lysine 6-acetyltransferase activity, acetyl-CoA:N6-hydroxy-L-lysine 6-acetyltransferase activity Sources: EC:2.3.1.102, RHEA:22388 Definition: Catalysis of the reaction: N(6)-hydroxy-L-lysine + acetyl-CoA = N(6)-acetyl-N(6)-hydroxy-L-lysine + CoA.